{
  "gene": "UniProtKB:Q86WK6",
  "gene_symbol": "AMIGO1",
  "term_id": "GO:0007157",
  "gene_name": "Amphoterin-induced protein 1",
  "term_label": "heterophilic cell-cell adhesion"
}